{
  "term_label": "regulation of cell shape",
  "gene": "UniProtKB:P60763",
  "gene_symbol": "RAC3",
  "term_id": "GO:0008360",
  "gene_name": "Ras-related C3 botulinum toxin substrate 3"
}